{
  "gene_name": "Peptidyl-prolyl cis-trans isomerase FKBP1B",
  "gene_symbol": "FKBP1B",
  "term_label": "regulation of ryanodine-sensitive calcium-release channel activity",
  "term_id": "GO:0060314",
  "gene": "UniProtKB:P68106"
}